{
  "gene": "UniProtKB:Q8N2U9",
  "term_label": "phospholipid translocation",
  "gene_symbol": "SLC66A2",
  "term_id": "GO:0045332",
  "gene_name": "Solute carrier family 66 member 2"
}